cell population proliferation [GO:0008283] (biological process) Definition: The multiplication or reproduction of cells, resulting in the expansion of a cell population. Note: This term was moved out from being a child of 'cellular process' because it is a cell population-level process, and cellular processes are restricted to those processes that involve individual cells. Also note that this term is intended to be used for the proliferation of cells within a multicellular organism, not for the expansion of a population of single-celled organisms. Subtypes: inner cell mass cell proliferation [GO:0001833], GO:0001834, mammary stem cell proliferation [GO:0002174], growth plate cartilage chondrocyte proliferation [GO:0003419], GO:0010463, glial cell proliferation [GO:0014009], muscle cell proliferation [GO:0033002], GO:0033687, hemocyte proliferation [GO:0035172], GO:0035726, cell proliferation involved in compound eye morphogenesis [GO:0035736], chondrocyte proliferation [GO:0035988], germ cell proliferation [GO:0036093], germ-line cyst formation [GO:0048134], fibroblast proliferation [GO:0048144], epithelial cell proliferation [GO:0050673], myoblast proliferation [GO:0051450], cell proliferation involved in embryonic placenta development [GO:0060722], cell proliferation involved in heart morphogenesis [GO:0061323], neural precursor cell proliferation [GO:0061351], fat cell proliferation [GO:0070341], leukocyte proliferation [GO:0070661], hair follicle cell proliferation [GO:0071335], cell proliferation in bone marrow [GO:0071838], stem cell proliferation [GO:0072089], cell proliferation involved in kidney development [GO:0072111], GO:0090255, chorionic trophoblast cell proliferation [GO:0097360], Leydig cell proliferation [GO:0160024], GO:2000793 Relationships: is a type of cellular process [GO:0009987] Sources: GOC:mah, GOC:mb Regulation: positively regulated by GO:0008284; negatively regulated by negative regulation of cell population proliferation [GO:0008285]; regulated by regulation of cell population proliferation [GO:0042127] Also known as: cell proliferation